{
  "term_id": "UNKNOWN:0003",
  "gene_name": "Putative transmenbrane protein RNF32-DT",
  "gene": "UniProtKB:Q8NI28",
  "gene_symbol": "RNF32-DT",
  "term_label": "Unknown cellular component"
}